{
  "term_label": "nucleus",
  "term_id": "GO:0005634",
  "gene": "UniProtKB:P23771",
  "gene_name": "Trans-acting T-cell-specific transcription factor GATA-3",
  "gene_symbol": "GATA3"
}